symbiont-mediated suppression of host inflammasome-mediated signal transduction [GO:0141081] (biological process) Relationships: is a type of symbiont-mediated suppression of cytoplasmic pattern recognition receptor signaling pathway [GO:0039537] Definition: A process in which a symbiont interferes with, inhibits or stops an inflammasome-mediated signal transduction pathway in the host organism by interfering with its normal execution. The host is defined as the larger of the organisms involved in a symbiotic interaction. References: PMID:26687278, PMID:27214553, PMID:29061850, PMID:34324582, PMID:36227980 Also known as: perturbation of host inflammasome-mediated signal transduction